{
  "gene": "UniProtKB:Q16720",
  "term_id": "GO:0005388",
  "gene_symbol": "ATP2B3",
  "gene_name": "Plasma membrane calcium-transporting ATPase 3",
  "term_label": "P-type calcium transporter activity"
}